{
  "term_label": "Cajal body organization",
  "gene_symbol": "WRAP53",
  "term_id": "GO:0030576",
  "gene": "UniProtKB:Q9BUR4",
  "gene_name": "Telomerase Cajal body protein 1"
}